{
  "gene": "UniProtKB:O15239",
  "term_label": "Unknown biological process",
  "gene_symbol": "NDUFA1",
  "term_id": "UNKNOWN:0002",
  "gene_name": "NADH dehydrogenase [ubiquinone] 1 alpha subcomplex subunit 1"
}